2,3-dihydroxybenzoate 2,3-dioxygenase activity [GO:0047072] (molecular function) Definition: Catalysis of the reaction: 2,3-dihydroxybenzoate + O2 = 2-carboxy-cis,cis-muconate + 2 H+. Also known as: 2,3-dihydroxybenzoate 2,3-oxygenase activity, 2,3-dihydroxybenzoate:oxygen 2,3-oxidoreductase (decyclizing) Relationships: is a type of GO:0016702 Sources: EC:1.13.11.28, RHEA:15369